hematopoietic stem cell homeostasis [GO:0061484] (BP) Definition: Any biological process involved in the maintenance of the steady-state number of hematopoietic stem cells within a population of cells. References: PMID:21508411 Sources: GOC:dph Relationships: is a type of homeostasis of number of cells [GO:0048872]